positive regulation of purine nucleobase metabolic process [GO:0045983] (biological process) Definition: Any process that activates or increases the frequency, rate or extent of the chemical reactions and pathways involving purine bases. Also known as: positive regulation of purine base metabolic process, positive regulation of purine base metabolism, up regulation of purine base metabolic process, up-regulation of purine base metabolic process, upregulation of purine base metabolic process, activation of purine base metabolic process, stimulation of purine base metabolic process Sources: GOC:go_curators Relationships: is a type of GO:0006141; is a type of GO:0062013; positively regulates purine nucleobase metabolic process [GO:0006144]